{
  "gene": "UniProtKB:Q6NWY9",
  "term_id": "GO:0005685",
  "gene_symbol": "PRPF40B",
  "term_label": "U1 snRNP",
  "gene_name": "Pre-mRNA-processing factor 40 homolog B"
}